{
  "gene_name": "Exosome complex component RRP46",
  "gene": "UniProtKB:Q9NQT4",
  "term_id": "GO:0071028",
  "gene_symbol": "EXOSC5",
  "term_label": "nuclear mRNA surveillance"
}